renal control of peripheral vascular resistance involved in regulation of systemic arterial blood pressure [GO:0003072] (biological process) Relationships: is a type of renal system process involved in regulation of systemic arterial blood pressure [GO:0003071] Also known as: regulation of systemic arterial blood pressure by renal control of peripheral vascular resistance, renal regulation of systemic arterial blood pressure by control of peripheral vascular resistance Definition: The renal process that modulates the force with which blood travels through the circulatory system, by impeding blood flow through the peripheral vasculature. Subtypes: GO:0002034, renal vasodilation of the peripheral vascular system involved in regulation of systemic arterial blood pressure [GO:0003075] Sources: GOC:mtg_cardio